{
  "gene_name": "Kelch-like protein 35",
  "gene": "UniProtKB:Q6PF15",
  "gene_symbol": "KLHL35",
  "term_id": "GO:0031463",
  "term_label": "Cul3-RING ubiquitin ligase complex"
}